cellular response to kainic acid [GO:1904374] (biological process) Relationships: is a type of cellular response to amino acid stimulus [GO:0071230]; is a type of cellular response to nitrogen compound [GO:1901699]; is a type of cellular response to oxygen-containing compound [GO:1901701]; is a type of GO:1904373 Definition: Any process that results in a change in state or activity of a cell (in terms of movement, secretion, enzyme production, gene expression, etc.) as a result of a kainic acid stimulus. References: PMID:17443789 Sources: GOC:TermGenie, GO_REF:0000071